{
  "term_label": "Unknown biological process",
  "gene_name": "Heparan sulfate glucosamine 3-O-sulfotransferase 4",
  "gene_symbol": "HS3ST4",
  "gene": "UniProtKB:Q9Y661",
  "term_id": "UNKNOWN:0002"
}